term tracker item [IAO:0000233] (external)